5-aminolevulinic acid transmembrane transporter activity [GO:0140485] (molecular function) Definition: Enables the transfer of 5-aminolevulinic acid from one side of a membrane to the other. References: PMID:31989647 Relationships: is a type of monocarboxylic acid transmembrane transporter activity [GO:0008028]; is a type of amino acid transmembrane transporter activity [GO:0015171]